nitrilotriacetate monooxygenase activity [GO:0018529] (molecular function) Sources: RHEA:31359 Definition: Catalysis of the reaction: nitrilotriacetate + FMNH2 + O2 = aminodiacetate + FMN + glyoxylate + H2O. Relationships: is a type of oxidoreductase activity, acting on paired donors, with incorporation or reduction of molecular oxygen, reduced flavin or flavoprotein as one donor, and incorporation of one atom of oxygen [GO:0016712]